{
  "gene_symbol": "RPS6KA6",
  "gene_name": "Ribosomal protein S6 kinase alpha-6",
  "term_id": "GO:0005737",
  "gene": "UniProtKB:Q9UK32",
  "term_label": "cytoplasm"
}